{
  "gene": "UniProtKB:Q8NBZ7",
  "term_id": "UNKNOWN:0002",
  "gene_symbol": "UXS1",
  "gene_name": "UDP-glucuronic acid decarboxylase 1",
  "term_label": "Unknown biological process"
}